{
  "term_label": "GTPase activator activity",
  "term_id": "GO:0005096",
  "gene_name": "ADP-ribosylation factor GTPase-activating protein 1",
  "gene": "UniProtKB:Q8N6T3",
  "gene_symbol": "ARFGAP1"
}